{
  "term_id": "GO:0005634",
  "gene_symbol": "PPP2R5B",
  "gene_name": "Serine_threonine-protein phosphatase 2A 56 kDa regulatory subunit beta isoform",
  "term_label": "nucleus",
  "gene": "UniProtKB:Q15173"
}